ITP binding [GO:1901641] (MF) Sources: GOC:TermGenie Definition: Binding to ITP. Relationships: is a type of GO:0032555; is a type of purine ribonucleoside triphosphate binding [GO:0035639]